{
  "term_label": "adenylate cyclase-activating G protein-coupled receptor signaling pathway",
  "gene": "UniProtKB:P43115",
  "term_id": "GO:0007189",
  "gene_symbol": "PTGER3",
  "gene_name": "Prostaglandin E2 receptor EP3 subtype"
}